purine nucleoside triphosphate biosynthetic process [GO:0009145] (biological process) Sources: GOC:go_curators, ISBN:0198506732 Subtypes: purine ribonucleoside triphosphate biosynthetic process [GO:0009206], GO:0009216 Relationships: is a type of GO:0009142; is a type of purine nucleoside triphosphate metabolic process [GO:0009144] Also known as: purine nucleoside triphosphate anabolism, purine nucleoside triphosphate biosynthesis, purine nucleoside triphosphate formation, purine nucleoside triphosphate synthesis Definition: The chemical reactions and pathways resulting in the formation of purine nucleoside triphosphate, a compound consisting of a purine base linked to a ribose or deoxyribose sugar esterified with triphosphate on the sugar.